{
  "term_id": "UNKNOWN:0003",
  "gene_name": "RNA-binding E3 ubiquitin-protein ligase MEX3C",
  "gene_symbol": "MEX3C",
  "gene": "UniProtKB:Q5U5Q3",
  "term_label": "Unknown cellular component"
}